{
  "term_id": "UNKNOWN:0003",
  "term_label": "Unknown cellular component",
  "gene_name": "Zinc finger protein SNAI3",
  "gene_symbol": "SNAI3",
  "gene": "UniProtKB:Q3KNW1"
}